{
  "term_label": "CCR chemokine receptor binding",
  "gene_symbol": "CCL4",
  "gene": "UniProtKB:P13236",
  "term_id": "GO:0048020",
  "gene_name": "C-C motif chemokine 4"
}